{
  "gene": "UniProtKB:Q9NZL4",
  "gene_name": "Hsp70-binding protein 1",
  "gene_symbol": "HSPBP1",
  "term_id": "GO:0000774",
  "term_label": "adenyl-nucleotide exchange factor activity"
}